bisdemethoxycurcumin synthase activity [GO:0102452] (molecular function) Definition: Catalysis of the reaction: 2 4-coumaryl-CoA + malonyl-CoA + H2O + H+ = 3 coenzyme A + bisdemethoxycurcumin + 2 carbon dioxide. Sources: EC:2.3.1.211, GOC:pz Relationships: is a type of acyltransferase activity, transferring groups other than amino-acyl groups [GO:0016747]